L-histidine transmembrane transport from lysosomal lumen to cytosol [GO:1904918] (biological process) References: PMID:22822152 Sources: GOC:TermGenie, GOC:kmv, GO_REF:0000078 Relationships: is a type of amino acid transmembrane export from vacuole [GO:0032974]; is a type of L-histidine transmembrane transport [GO:0089709]; is a type of transmembrane transport from lysosomal lumen to cytosol [GO:0170063] Also known as: transmembrane L-histidine transport from lysosomal lumen to cytosol Definition: The directed movement of L-histidine from the lysosomal lumen across the lysosomal membrane and into the cytosol.